{
  "gene_name": "RNA-binding protein Nova-1",
  "term_label": "nucleus",
  "term_id": "GO:0005634",
  "gene": "UniProtKB:P51513",
  "gene_symbol": "NOVA1"
}